mammillotegmental axonal tract development [GO:0061376] (biological process) Definition: The process in which the mammillotegmental tract progresses over time, from its formation to the mature structure. The mammillotegmental tract is the collection of axons that connects the ventral diencephalon to the tegmentum and pons. References: PMID:10662642 Sources: GOC:dph, GOC:yaf Relationships: is a type of GO:0048856; is part of mammillary axonal complex development [GO:0061373]